{
  "gene": "UniProtKB:Q8IWT6",
  "gene_name": "Volume-regulated anion channel subunit LRRC8A",
  "term_label": "monoatomic anion transmembrane transport",
  "gene_symbol": "LRRC8A",
  "term_id": "GO:0098656"
}